{
  "term_id": "GO:0051156",
  "gene_name": "Glucose-6-phosphatase catalytic subunit 1",
  "gene_symbol": "G6PC1",
  "gene": "UniProtKB:P35575",
  "term_label": "glucose 6-phosphate metabolic process"
}